{
  "gene": "UniProtKB:Q9BTC8",
  "term_label": "transcription corepressor activity",
  "term_id": "GO:0003714",
  "gene_symbol": "MTA3",
  "gene_name": "Metastasis-associated protein MTA3"
}